regulation of NAD metabolic process [GO:1902688] (biological process) Relationships: is a type of regulation of purine nucleotide metabolic process [GO:1900542]; regulates NAD+ metabolic process [GO:0019674] Definition: Any process that modulates the frequency, rate or extent of NAD metabolic process. Also known as: regulation of NAD (oxidized) metabolic process, regulation of NAD (oxidized) metabolism, regulation of NAD metabolism, regulation of nicotinamide adenine dinucleotide metabolic process, regulation of nicotinamide adenine dinucleotide metabolism, regulation of oxidized NAD metabolic process, regulation of oxidized NAD metabolism, regulation of oxidized nicotinamide adenine dinucleotide metabolic process, regulation of oxidized nicotinamide adenine dinucleotide metabolism, regulation of NAD phosphorylation and dephosphorylation References: PMID:19846558 Sources: GOC:TermGenie, GOC:di, GO_REF:0000058 Subtypes: GO:1902689, positive regulation of NAD metabolic process [GO:1902690], GO:1905012